{
  "gene": "UniProtKB:O60674",
  "gene_symbol": "JAK2",
  "term_label": "cytosol",
  "gene_name": "Tyrosine-protein kinase JAK2",
  "term_id": "GO:0005829"
}